N-terminal protein amino acid methylation [GO:0006480] (biological process) Relationships: is a type of protein methylation [GO:0006479]; is a type of GO:0031365 Definition: The methylation of the N-terminal amino acid of a protein. Sources: GOC:ai Subtypes: N-terminal peptidyl-alanine methylation [GO:0018011], N-terminal peptidyl-glycine methylation [GO:0018013], N-terminal peptidyl-proline methylation [GO:0035568], N-terminal peptidyl-serine methylation [GO:0035570]